{
  "gene_name": "tRNA N(3)-methylcytidine methyltransferase METTL2A",
  "gene": "UniProtKB:Q96IZ6",
  "term_label": "Unknown biological process",
  "term_id": "UNKNOWN:0002",
  "gene_symbol": "METTL2A"
}